{
  "term_id": "UNKNOWN:0003",
  "gene_symbol": "HCST",
  "term_label": "Unknown cellular component",
  "gene_name": "Hematopoietic cell signal transducer",
  "gene": "UniProtKB:Q9UBK5"
}